{
  "gene_name": "Ceramide glucosyltransferase",
  "gene": "UniProtKB:Q16739",
  "gene_symbol": "UGCG",
  "term_id": "GO:0008120",
  "term_label": "ceramide glucosyltransferase activity"
}